{
  "gene": "UniProtKB:P17302",
  "gene_name": "Gap junction alpha-1 protein",
  "term_label": "cell communication by electrical coupling",
  "gene_symbol": "GJA1",
  "term_id": "GO:0010644"
}